snoRNA transcription by RNA polymerase III [GO:0001014] (biological process) Definition: The synthesis of small nucleolar RNA (snoRNA) from a DNA template by RNA polymerase III, originating at a type 2 RNA polymerase III promoter. Sources: GOC:txnOH Also known as: snoRNA transcription from a type 2 RNA polymerase III promoter Relationships: is a type of transcription by RNA polymerase III [GO:0006383]; is a type of sno(s)RNA transcription [GO:0009302]